{
  "term_id": "GO:0006612",
  "gene": "UniProtKB:Q5QGT7",
  "gene_symbol": "RTP2",
  "gene_name": "Receptor-transporting protein 2",
  "term_label": "protein targeting to membrane"
}